regulation of protein lipidation [GO:1903059] (biological process) References: PMID:21909394 Sources: GOC:TermGenie, GOC:rph, GO_REF:0000058 Subtypes: regulation of N-terminal protein palmitoylation [GO:0060254], regulation of peptidyl-L-cysteine S-palmitoylation [GO:1902662], negative regulation of protein lipidation [GO:1903060], GO:1903061 Definition: Any process that modulates the frequency, rate or extent of protein lipidation. Relationships: is a type of GO:0010556; is a type of regulation of protein modification process [GO:0031399]; is a type of regulation of lipoprotein metabolic process [GO:0050746]; regulates protein lipidation [GO:0006497] Also known as: regulation of lipid:protein modification, regulation of protein amino acid lipidation